{
  "term_label": "mRNA regulatory element binding translation repressor activity",
  "term_id": "GO:0000900",
  "gene": "UniProtKB:Q17RY0",
  "gene_name": "Cytoplasmic polyadenylation element-binding protein 4",
  "gene_symbol": "CPEB4"
}